{
  "gene": "UniProtKB:Q6ZUV0",
  "term_id": "GO:0006637",
  "gene_symbol": "ACOT7L",
  "term_label": "acyl-CoA metabolic process",
  "gene_name": "Putative cytosolic acyl coenzyme A thioester hydrolase-like"
}